{
  "term_id": "UNKNOWN:0003",
  "term_label": "Unknown cellular component",
  "gene_symbol": "KRTAP12-4",
  "gene_name": "Keratin-associated protein 12-4",
  "gene": "UniProtKB:P60329"
}